{
  "term_id": "GO:0008284",
  "gene": "UniProtKB:Q14627",
  "term_label": "positive regulation of cell population proliferation",
  "gene_symbol": "IL13RA2",
  "gene_name": "Interleukin-13 receptor subunit alpha-2"
}